{
  "term_id": "GO:0043565",
  "gene_symbol": "RAG1",
  "term_label": "sequence-specific DNA binding",
  "gene_name": "V(D)J recombination-activating protein 1",
  "gene": "UniProtKB:P15918"
}